{
  "gene_name": "Putative ATP-dependent RNA helicase DDX11-like protein 8",
  "gene_symbol": "DDX11L8",
  "term_id": "GO:0003678",
  "term_label": "DNA helicase activity",
  "gene": "UniProtKB:A8MPP1"
}